{
  "gene_name": "CD99 antigen",
  "term_label": "positive regulation of neutrophil extravasation",
  "term_id": "GO:2000391",
  "gene_symbol": "CD99",
  "gene": "UniProtKB:P14209"
}